{
  "gene_name": "Reticulon-3",
  "term_label": "postsynaptic density",
  "term_id": "GO:0014069",
  "gene": "UniProtKB:O95197",
  "gene_symbol": "RTN3"
}